{
  "gene": "UniProtKB:Q00587",
  "gene_name": "Cdc42 effector protein 1",
  "term_id": "GO:0031274",
  "gene_symbol": "CDC42EP1",
  "term_label": "positive regulation of pseudopodium assembly"
}